TRIF-dependent toll-like receptor signaling pathway [GO:0035666] (biological process) Subtypes: TRIF-dependent toll-like receptor 4 signaling pathway [GO:0035667] Definition: The series of molecular signals initiated by a ligand binding to a toll-like receptor where the TRIF adaptor mediates transduction of the signal. Toll-like receptors directly bind pattern motifs from a variety of microbial sources to initiate an innate immune response. Also known as: TRIF-dependent TLR signaling pathway, TRIF-dependent toll-like receptor signalling pathway, Toll/IL-1 receptor (TIR) domain-containing adaptor-dependent TLR signaling pathway References: PMID:12855817 Sources: GOC:BHF Relationships: is a type of MyD88-independent toll-like receptor signaling pathway [GO:0002756]